{
  "term_id": "GO:0008237",
  "term_label": "metallopeptidase activity",
  "gene_name": "COP9 signalosome complex subunit 5",
  "gene": "UniProtKB:Q92905",
  "gene_symbol": "COPS5"
}